L-glutamate catabolic process to ornithine [GO:0019555] (biological process) Definition: The chemical reactions and pathways resulting in the breakdown of L-glutamate into other compounds, including ornithine. Also known as: glutamate breakdown to ornithine, glutamate degradation to ornithine Relationships: is_a L-glutamate catabolic process [GO:0006538]; is a type of ornithine metabolic process [GO:0006591] Sources: GOC:go_curators